ferredoxin-NAD+ reductase activity [GO:0008860] (molecular function) Definition: Catalysis of the reaction: 2 reduced [2Fe-2S]-[ferredoxin] + NAD+ + H+ = 2 oxidized [2Fe-2S]-[ferredoxin] + NADH. Relationships: is a type of ferredoxin-[NAD(P)H] reductase activity [GO:0008937] Also known as: ferredoxin-NAD reductase activity, NAD-ferredoxin reductase activity, NADH flavodoxin oxidoreductase activity, NADH-ferredoxin oxidoreductase activity, NADH-ferredoxin reductase activity, NADH-ferredoxinNAP reductase (component of naphthalene dioxygenase multicomponent enzyme system), NADH-ferredoxinTOL reductase (component of toluene dioxygenase), NADH2-ferredoxin oxidoreductase activity, ferredoxin-linked NAD reductase activity, ferredoxin-nicotinamide adenine dinucleotide reductase activity, ferredoxin:NAD+ oxidoreductase activity, reductase, reduced nicotinamide adenine dinucleotide-ferredoxin Sources: RHEA:16521